{
  "gene_name": "Signal peptide peptidase-like 2A",
  "term_id": "GO:0042500",
  "gene_symbol": "SPPL2A",
  "gene": "UniProtKB:Q8TCT8",
  "term_label": "aspartic endopeptidase activity, intramembrane cleaving"
}